negative regulation of cytokinin-activated signaling pathway [GO:0080037] (biological process) Relationships: is a type of negative regulation of signal transduction [GO:0009968]; is a type of GO:0080036; negatively regulates cytokinin-activated signaling pathway [GO:0009736] Also known as: negative regulation of cytokinin mediated signalling, negative regulation of cytokinin mediated signaling pathway References: PMID:14973166 Sources: GOC:dhl Definition: Any process that stops, prevents, or reduces the frequency, rate or extent of cytokinin signaling.